{
  "gene_name": "MICOS complex subunit MIC25",
  "term_id": "GO:0006974",
  "gene": "UniProtKB:Q9BRQ6",
  "term_label": "DNA damage response",
  "gene_symbol": "CHCHD6"
}